{
  "term_label": "plasma membrane",
  "gene": "UniProtKB:Q5XXA6",
  "gene_symbol": "ANO1",
  "term_id": "GO:0005886",
  "gene_name": "Anoctamin-1"
}